{
  "gene_name": "60 kDa lysophospholipase",
  "term_label": "Unknown cellular component",
  "term_id": "UNKNOWN:0003",
  "gene_symbol": "ASPG",
  "gene": "UniProtKB:Q86U10"
}